{
  "gene_symbol": "AQP7P3",
  "gene": "UniProtKB:A6NL99",
  "gene_name": "Putative aquaporin-7-like protein 3",
  "term_id": "UNKNOWN:0001",
  "term_label": "Unknown molecular function"
}